{
  "gene_symbol": "WIPI2",
  "term_label": "protein localization to phagophore assembly site",
  "gene": "UniProtKB:Q9Y4P8",
  "term_id": "GO:0034497",
  "gene_name": "WD repeat domain phosphoinositide-interacting protein 2"
}